{
  "gene": "UniProtKB:Q96MI9",
  "gene_symbol": "AGBL1",
  "term_label": "tubulin binding",
  "term_id": "GO:0015631",
  "gene_name": "Cytosolic carboxypeptidase 4"
}